{
  "gene_name": "Putative tumor antigen NA88-A",
  "term_label": "Unknown molecular function",
  "term_id": "UNKNOWN:0001",
  "gene": "UniProtKB:P0C5K6",
  "gene_symbol": "VENTXP1"
}